dolichyl diphosphate biosynthetic process [GO:0006489] (biological process) Relationships: is a type of phospholipid biosynthetic process [GO:0008654]; is part of dolichol-linked oligosaccharide biosynthetic process [GO:0006488] Sources: ISBN:0198506732 Definition: The chemical reactions and pathways resulting in the formation of dolichyl diphosphate, a diphosphorylated dolichol derivative. Also known as: dolichyl diphosphate anabolism, dolichyl diphosphate biosynthesis, dolichyl diphosphate formation, dolichyl diphosphate synthesis